circadian sleep/wake cycle [GO:0042745] (biological process) Regulation: regulated by GO:0042749 Definition: The cycle from wakefulness through an orderly succession of sleep states and stages that occurs on an approximately 24 hour rhythm. References: PMID:26947521, PMID:33537937 Sources: GOC:jl Relationships: is a type of circadian behavior [GO:0048512]